{
  "term_id": "GO:0051968",
  "gene_name": "Voltage-dependent calcium channel gamma-2 subunit",
  "term_label": "positive regulation of synaptic transmission, glutamatergic",
  "gene_symbol": "CACNG2",
  "gene": "UniProtKB:Q9Y698"
}